positive regulation of chemokine-mediated signaling pathway [GO:0070101] (biological process) Subtypes: GO:1903082 Also known as: positive regulation of chemokine-mediated signalling pathway Relationships: is a type of GO:0001961; is a type of positive regulation of G protein-coupled receptor signaling pathway [GO:0045745]; is a type of GO:0070099; positively regulates chemokine-mediated signaling pathway [GO:0070098] Definition: Any process that increases the rate, frequency or extent of a chemokine-mediated signaling pathway. Sources: GOC:mah